{
  "term_id": "GO:0006888",
  "term_label": "endoplasmic reticulum to Golgi vesicle-mediated transport",
  "gene": "UniProtKB:Q9HCU5",
  "gene_symbol": "PREB",
  "gene_name": "Prolactin regulatory element-binding protein"
}